{
  "term_id": "UNKNOWN:0003",
  "gene": "UniProtKB:Q9BYE2",
  "gene_symbol": "TMPRSS13",
  "gene_name": "Transmembrane protease serine 13",
  "term_label": "Unknown cellular component"
}